{
  "term_label": "regulation of transcription by RNA polymerase II",
  "gene": "UniProtKB:Q9UQR1",
  "gene_name": "Zinc finger protein 148",
  "term_id": "GO:0006357",
  "gene_symbol": "ZNF148"
}